{
  "gene": "UniProtKB:P0DN81",
  "term_label": "olfactory receptor activity",
  "term_id": "GO:0004984",
  "gene_symbol": "OR13C7",
  "gene_name": "Olfactory receptor 13C7"
}